{
  "gene_name": "Ribosome-releasing factor 2, mitochondrial",
  "gene": "UniProtKB:Q969S9",
  "gene_symbol": "GFM2",
  "term_label": "ribosome disassembly",
  "term_id": "GO:0032790"
}